{
  "gene_name": "Telomerase RNA component interacting RNase",
  "gene": "UniProtKB:Q9BQ61",
  "gene_symbol": "TRIR",
  "term_id": "UNKNOWN:0002",
  "term_label": "Unknown biological process"
}